{
  "gene": "UniProtKB:O43524",
  "gene_name": "Forkhead box protein O3",
  "term_id": "GO:0005634",
  "term_label": "nucleus",
  "gene_symbol": "FOXO3"
}